tricarboxylic acid cycle [GO:0006099] (biological process) Relationships: is_a primary metabolic process [GO:0044238]; is part of GO:0009060 Definition: A nearly universal metabolic pathway in which the acetyl group of acetyl coenzyme A is effectively oxidized to two CO2 and four pairs of electrons are transferred to coenzymes. The acetyl group combines with oxaloacetate to form citrate, which undergoes successive transformations to isocitrate, 2-oxoglutarate, succinyl-CoA, succinate, fumarate, malate, and oxaloacetate again, thus completing the cycle. In eukaryotes the tricarboxylic acid is confined to the mitochondria. See also glyoxylate cycle. Also known as: Krebs cycle, TCA cycle, citric acid cycle, oxidative TCA cycle Sources: ISBN:0198506732